{
  "gene": "UniProtKB:Q6ZNL6",
  "gene_symbol": "FGD5",
  "term_label": "cytoplasm",
  "term_id": "GO:0005737",
  "gene_name": "FYVE, RhoGEF and PH domain-containing protein 5"
}